cargo receptor ligand activity [GO:0140355] (molecular function) Relationships: is a type of protein binding [GO:0005515] Also known as: cargo References: PMID:15797858 Definition: The activity of a gene product that interacts with a cargo receptor and initiates endocytosis.